{
  "term_label": "inner ear development",
  "gene_symbol": "SOX2",
  "term_id": "GO:0048839",
  "gene_name": "Transcription factor SOX-2",
  "gene": "UniProtKB:P48431"
}